{
  "gene_name": "Dickkopf-related protein 1",
  "term_id": "GO:0005615",
  "gene_symbol": "DKK1",
  "gene": "UniProtKB:O94907",
  "term_label": "extracellular space"
}